{
  "gene_name": "Uncharacterized protein C2orf74",
  "term_label": "Unknown molecular function",
  "gene_symbol": "C2orf74",
  "term_id": "UNKNOWN:0001",
  "gene": "UniProtKB:A8MZ97"
}